glycosome organization [GO:0106233] (biological process) Relationships: is a type of GO:0006996 Definition: A process that is carried out at the cellular level which results in the assembly, arrangement of constituent parts, or disassembly of a glycosome, a membrane-bounded organelle found in organisms from the order Kinetoplastida that houses the enzymes of glycolysis. Also known as: glycosome organisation, glycosome biogenesis, glycosome organization and biogenesis References: PMID:15539076, PMID:28426655, PMID:31341002, PMID:8056787 Sources: GOC:ach